chrysobactin transmembrane transporter activity [GO:0042933] (molecular function) Also known as: chrysobactin transporter activity Relationships: is a type of monocarboxylic acid transmembrane transporter activity [GO:0008028]; is a type of GO:0015343; is a type of alcohol transmembrane transporter activity [GO:0015665]; is a type of GO:0071916; is part of chrysobactin transport [GO:0042932] References: PMID:8837459 Sources: GOC:jl Definition: Enables the directed movement of the siderophore chrysobactin (alpha-N-(2,3-dihydroxybenzoyl)-D-lysyl-L-serine) from one side of a membrane to the other.